inulin fructotransferase (DFA-I-forming) activity [GO:0033997] (MF) Sources: EC:4.2.2.17 Definition: Catalysis of the reaction: [(2->1)-beta-D-fructosyl](n) = [(2->1)-beta-D-fructosyl](n-1) + alpha-D-fructofuranose-beta-D-fructofuranose 1,2':1,2'-dianhydride. This reaction is the production of alpha-D-fructofuranose beta-D-fructofuranose 1,2':2,1'-dianhydride (DFA I) by successively eliminating the diminishing (2->1)-beta-D-fructan (inulin) chain from the terminal D-fructosyl-D-fructosyl disaccharide. Also known as: 2,1-beta-D-fructan lyase (alpha-D-fructofuranose-beta-D-fructofuranose-1,2':2,1'-dianhydride-forming) activity, inulin D-fructosyl-D-fructosyltransferase (1,2':1',2-dianhydride-forming) activity, inulin D-fructosyl-D-fructosyltransferase (forming alpha-D-fructofuranose beta-D-fructofuranose 1,2':1',2-dianhydride) activity, inulin fructotransferase (DFA-I-producing) activity, inulin fructotransferase (depolymerizing, difructofuranose-1,2':2',1-dianhydride-forming) activity Relationships: is_a GO:0016837